{
  "gene_name": "Lymphocyte antigen 6 family member G6E",
  "term_id": "GO:0030549",
  "term_label": "acetylcholine receptor activator activity",
  "gene_symbol": "LY6G6E",
  "gene": "UniProtKB:A0A0B4J1T7"
}